glyceryl-ether monooxygenase activity [GO:0050479] (molecular function) Relationships: is a type of oxidoreductase activity, acting on paired donors, with incorporation or reduction of molecular oxygen, reduced pteridine as one donor, and incorporation of one atom of oxygen [GO:0016714] Definition: Catalysis of the reaction: 1-alkyl-sn-glycerol + O2 + (tetrahydrobiopterin/tetrahydropteridine) = 1-hydroxyalkyl-sn-glycerol + H2O + (dihydrobiopterin/dihydropteridine). Sources: EC:1.14.16.5, MetaCyc:GLYCERYL-ETHER-MONOOXYGENASE-RXN Also known as: 1-alkyl-sn-glycerol,tetrahydrobiopterin:oxygen oxidoreductase activity, O-alkylglycerol monooxygenase activity, alkylglycerol monooxygenase activity, glyceryl ether oxygenase activity, glyceryl etherase activity, glyceryl-ether cleaving enzyme activity